{
  "term_id": "GO:0000785",
  "gene_name": "Estrogen receptor beta",
  "gene_symbol": "ESR2",
  "gene": "UniProtKB:Q92731",
  "term_label": "chromatin"
}